{
  "gene": "UniProtKB:Q8N4L2",
  "term_label": "late endosome membrane",
  "term_id": "GO:0031902",
  "gene_name": "Type 2 phosphatidylinositol 4,5-bisphosphate 4-phosphatase",
  "gene_symbol": "PIP4P2"
}